{
  "gene_symbol": "SLC6A9",
  "term_label": "sodium ion transmembrane transport",
  "term_id": "GO:0035725",
  "gene_name": "Sodium- and chloride-dependent glycine transporter 1",
  "gene": "UniProtKB:P48067"
}